{
  "gene_name": "Exosome complex exonuclease RRP44",
  "term_id": "GO:0016075",
  "term_label": "rRNA catabolic process",
  "gene_symbol": "DIS3",
  "gene": "UniProtKB:Q9Y2L1"
}